{
  "gene": "UniProtKB:A0A589",
  "gene_name": "T cell receptor beta variable 4-3",
  "term_label": "Unknown molecular function",
  "gene_symbol": "TRBV4-3",
  "term_id": "UNKNOWN:0001"
}